succinate:proton symporter activity [GO:0097434] (molecular function) References: PMID:1293882 Sources: GOC:al Relationships: is_a succinate transmembrane transporter activity [GO:0015141]; is a type of solute:proton symporter activity [GO:0015295] Also known as: succinate:hydrogen symporter activity Definition: Enables the transfer of a solute or solutes from one side of a membrane to the other according to the reaction: succinate(out) + H+(out) = succinate(in) + H+(in).